{
  "term_label": "Unknown biological process",
  "gene": "UniProtKB:P22061",
  "gene_name": "Protein-L-isoaspartate(D-aspartate) O-methyltransferase",
  "term_id": "UNKNOWN:0002",
  "gene_symbol": "PCMT1"
}